{
  "term_label": "peroxisomal membrane",
  "term_id": "GO:0005778",
  "gene_symbol": "PEX5",
  "gene": "UniProtKB:P50542",
  "gene_name": "Peroxisomal targeting signal 1 receptor"
}